P-TEFb complex [GO:0070691] (cellular component) Relationships: is a type of cyclin/CDK positive transcription elongation factor complex [GO:0008024] Also known as: Bur1/Bur2 complex, Sgv1/Bur2 complex, cyclin-dependent kinase 9 (Cdk9)-cyclin T1 complex, cyclin-dependent kinase 9 (Cdk9)-cyclin T2 complex, dimeric positive transcription elongation factor complex b Definition: A dimeric positive transcription elongation factor complex b that comprises a cyclin-dependent kinase containing the catalytic subunit, Cdk9, and a regulatory subunit, cyclin T. References: PMID:16721054, PMID:19328067 Sources: GOC:mah, GOC:vw, Wikipedia:P-TEFb